{
  "term_label": "Unknown molecular function",
  "gene_name": "WD repeat-containing protein 73",
  "gene_symbol": "WDR73",
  "term_id": "UNKNOWN:0001",
  "gene": "UniProtKB:Q6P4I2"
}